negative regulation of neutrophil mediated killing of gram-positive bacterium [GO:0070958] (biological process) Definition: Any process that decreases the frequency, rate or extent of the directed killing of a gram-positive bacterium by a neutrophil. Also known as: down regulation of neutrophil mediated killing of gram-positive bacterium, down-regulation of neutrophil mediated killing of gram-positive bacterium, downregulation of neutrophil mediated killing of gram-positive bacterium, inhibition of neutrophil mediated killing of gram-positive bacterium Sources: GOC:add, GOC:mah Relationships: is a type of GO:0070952; is a type of GO:0070956; negatively regulates neutrophil-mediated killing of gram-positive bacterium [GO:0070946]